{
  "gene_name": "rRNA methyltransferase 1, mitochondrial",
  "term_label": "mitochondrion",
  "term_id": "GO:0005739",
  "gene": "UniProtKB:Q6IN84",
  "gene_symbol": "MRM1"
}